{
  "gene": "UniProtKB:Q8TBE3",
  "gene_symbol": "FNDC9",
  "term_label": "Unknown molecular function",
  "term_id": "UNKNOWN:0001",
  "gene_name": "Fibronectin type III domain-containing protein 9"
}